{
  "term_id": "UNKNOWN:0001",
  "gene_symbol": "IGKV1-13",
  "term_label": "Unknown molecular function",
  "gene_name": "Immunoglobulin kappa variable 1-13",
  "gene": "UniProtKB:P0DP09"
}